negative regulation of crystal cell differentiation [GO:0042690] (biological process) Also known as: down regulation of crystal cell differentiation, down-regulation of crystal cell differentiation, downregulation of crystal cell differentiation, inhibition of crystal cell differentiation Sources: GOC:go_curators Definition: Any process that stops, prevents, or reduces the frequency, rate or extent of crystal cell differentiation. Relationships: is_a regulation of crystal cell differentiation [GO:0042689]; is a type of GO:0045611; negatively regulates crystal cell differentiation [GO:0042688]